{
  "term_label": "G protein-coupled purinergic nucleotide receptor activity",
  "gene_name": "Platelet-activating factor receptor",
  "term_id": "GO:0045028",
  "gene_symbol": "PTAFR",
  "gene": "UniProtKB:P25105"
}